{
  "term_id": "GO:0005886",
  "term_label": "plasma membrane",
  "gene": "UniProtKB:Q9H6S3",
  "gene_name": "Epidermal growth factor receptor kinase substrate 8-like protein 2",
  "gene_symbol": "EPS8L2"
}